{
  "gene_symbol": "B4GALT6",
  "gene": "UniProtKB:Q9UBX8",
  "gene_name": "Beta-1,4-galactosyltransferase 6",
  "term_id": "GO:0006688",
  "term_label": "glycosphingolipid biosynthetic process"
}